{
  "term_label": "early endosome",
  "gene_name": "Ribosomal protein S6 kinase delta-1",
  "term_id": "GO:0005769",
  "gene_symbol": "RPS6KC1",
  "gene": "UniProtKB:Q96S38"
}